cellular response to chemokine [GO:1990869] (biological process) References: PMID:11113082 Relationships: is a type of cellular response to cytokine stimulus [GO:0071345]; is a type of response to chemokine [GO:1990868] Definition: Any process that results in a change in state or activity of a cell (in terms of movement, secretion, enzyme production, gene expression, etc.) as a result of a chemokine stimulus.